{
  "gene_symbol": "MS4A18",
  "gene_name": "Membrane-spanning 4-domains subfamily A member 18",
  "gene": "UniProtKB:Q3C1V0",
  "term_label": "cell surface receptor signaling pathway",
  "term_id": "GO:0007166"
}